{
  "gene_name": "Zinc finger protein ZIC 3",
  "gene_symbol": "ZIC3",
  "gene": "UniProtKB:O60481",
  "term_id": "GO:0000981",
  "term_label": "DNA-binding transcription factor activity, RNA polymerase II-specific"
}